exit from reproductive diapause [GO:0071983] (biological process) Definition: The dormancy process that results in exit from reproductive diapause. Reproductive diapause is a form of diapause where the organism itself will remain fully active, including feeding and other routine activities, but the reproductive organs experience a tissue-specific reduction in metabolism, with characteristic triggering and releasing stimuli. Sources: GOC:mah Relationships: is_a GO:0071981